{
  "gene": "UniProtKB:P49910",
  "term_label": "regulation of transcription by RNA polymerase II",
  "gene_name": "Zinc finger protein 165",
  "term_id": "GO:0006357",
  "gene_symbol": "ZNF165"
}